{
  "gene_symbol": "TRH",
  "term_label": "Unknown biological process",
  "term_id": "UNKNOWN:0002",
  "gene": "UniProtKB:P20396",
  "gene_name": "Pro-thyrotropin-releasing hormone"
}